{
  "gene_name": "Neurogranin",
  "term_label": "Unknown biological process",
  "gene": "UniProtKB:Q92686",
  "gene_symbol": "NRGN",
  "term_id": "UNKNOWN:0002"
}